peptidase inhibitor complex [GO:1904090] (cellular component) Note: An example of this is Cystatin-A in human (UniProt symbol P01040) in PMID:20860624 (inferred from physical interaction). Subtypes: protease inhibitor complex [GO:0097179] Relationships: is a type of protein-containing complex [GO:0032991] References: PMID:20860624 Sources: GOC:TermGenie, GOC:bhm, GO_REF:0000088 Definition: A protein complex which is capable of peptidase inhibitor activity. Also known as: Cathepsin-B - cystatin-A complex